hydrolase activity, acting on acid carbon-phosphorus bonds [GO:0016827] (MF) Definition: Catalysis of the hydrolysis of any acid carbon-phosphorus bond. Sources: EC:3.11.-.- Relationships: is a type of hydrolase activity [GO:0016787] Subtypes: phosphonopyruvate hydrolase activity [GO:0033978], GO:0047400, phosphonoacetaldehyde hydrolase activity [GO:0050194]